{
  "gene_symbol": "LRRC8B",
  "gene": "UniProtKB:Q6P9F7",
  "gene_name": "Volume-regulated anion channel subunit LRRC8B",
  "term_label": "cyclic-GMP-AMP transmembrane import across plasma membrane",
  "term_id": "GO:0140361"
}